{
  "term_id": "GO:0016020",
  "gene_name": "Transmembrane protein 132C",
  "gene_symbol": "TMEM132C",
  "term_label": "membrane",
  "gene": "UniProtKB:Q8N3T6"
}